{
  "gene": "UniProtKB:Q96D53",
  "gene_symbol": "COQ8B",
  "term_label": "Unknown molecular function",
  "gene_name": "Atypical kinase COQ8B, mitochondrial",
  "term_id": "UNKNOWN:0001"
}